positive regulation of interleukin-1-mediated signaling pathway [GO:2000661] (biological process) Definition: Any process that activates or increases the frequency, rate or extent of interleukin-1-mediated signaling pathway. Sources: GOC:obol Also known as: positive regulation of IL-1-mediated signaling pathway, positive regulation of interleukin-1-mediated signalling pathway, positive regulation of IL-1 alpha-mediated signaling pathway, positive regulation of IL-1 beta-mediated signaling pathway, positive regulation of interleukin-1 alpha-mediated signaling pathway, positive regulation of interleukin-1 beta-mediated signaling pathway Relationships: is a type of GO:0001961; is a type of regulation of interleukin-1-mediated signaling pathway [GO:2000659]; positively regulates interleukin-1-mediated signaling pathway [GO:0070498]